{
  "gene_name": "Mucolipin-3",
  "term_label": "lysosomal membrane",
  "gene_symbol": "MCOLN3",
  "gene": "UniProtKB:Q8TDD5",
  "term_id": "GO:0005765"
}